{
  "term_label": "mitochondrion",
  "term_id": "GO:0005739",
  "gene": "UniProtKB:Q6UB28",
  "gene_name": "Methionine aminopeptidase 1D, mitochondrial",
  "gene_symbol": "METAP1D"
}